{
  "term_id": "GO:0016236",
  "gene": "UniProtKB:Q9H2M9",
  "term_label": "macroautophagy",
  "gene_name": "Rab3 GTPase-activating protein non-catalytic subunit",
  "gene_symbol": "RAB3GAP2"
}